type 2 angiotensin receptor binding [GO:0031703] (molecular function) Sources: GOC:mah, GOC:nln Also known as: AT2 receptor binding, type 2 angiotensin receptor ligand Definition: Binding to a type 2 angiotensin receptor. Relationships: is a type of angiotensin receptor binding [GO:0031701]